{
  "gene": "UniProtKB:Q8N100",
  "gene_symbol": "ATOH7",
  "term_id": "GO:0000981",
  "gene_name": "Transcription factor ATOH7",
  "term_label": "DNA-binding transcription factor activity, RNA polymerase II-specific"
}